{
  "gene_symbol": "SLC8A3",
  "term_id": "GO:0042383",
  "gene": "UniProtKB:P57103",
  "term_label": "sarcolemma",
  "gene_name": "Sodium_calcium exchanger 3"
}